{
  "gene_name": "Vacuolar protein sorting-associated protein 41 homolog",
  "gene_symbol": "VPS41",
  "gene": "UniProtKB:P49754",
  "term_label": "vacuolar transport",
  "term_id": "GO:0007034"
}